{
  "gene_symbol": "SPTSSA",
  "term_label": "serine palmitoyltransferase complex",
  "gene_name": "Serine palmitoyltransferase small subunit A",
  "term_id": "GO:0017059",
  "gene": "UniProtKB:Q969W0"
}